{
  "term_label": "P granule",
  "term_id": "GO:0043186",
  "gene_symbol": "PIWIL2",
  "gene_name": "Piwi-like protein 2",
  "gene": "UniProtKB:Q8TC59"
}